{
  "term_id": "UNKNOWN:0003",
  "gene": "UniProtKB:Q49AR2",
  "gene_name": "UPF0489 protein C5orf22",
  "gene_symbol": "C5orf22",
  "term_label": "Unknown cellular component"
}